{
  "term_label": "cholesterol catabolic process",
  "term_id": "GO:0006707",
  "gene_symbol": "CYP46A1",
  "gene_name": "Cholesterol 24-hydroxylase",
  "gene": "UniProtKB:Q9Y6A2"
}